beta-fructofuranosidase activity [GO:0004564] (molecular function) Subtypes: sucrose alpha-glucosidase activity [GO:0004575] Definition: Catalysis of the reaction: a fructofuranosylated fructofuranosyl acceptor + H2O = a non fructofuranosylated fructofuranosyl acceptor + a beta-D-fructofuranoside. Relationships: is a type of hydrolase activity, hydrolyzing O-glycosyl compounds [GO:0004553] Also known as: acid invertase activity, alkaline invertase activity, invertase activity, invertin activity, beta-D-fructofuranoside fructohydrolase activity, beta-fructosidase activity, beta-h-fructosidase activity, fructosylinvertase activity, glucosucrase activity, maxinvert L 1000 activity, saccharase activity Sources: EC:3.2.1.26, MetaCyc:RXN-9985